{
  "gene": "UniProtKB:P33681",
  "term_id": "GO:0009897",
  "gene_symbol": "CD80",
  "term_label": "external side of plasma membrane",
  "gene_name": "T-lymphocyte activation antigen CD80"
}